{
  "term_id": "UNKNOWN:0003",
  "gene_symbol": "SAA4",
  "gene": "UniProtKB:P35542",
  "term_label": "Unknown cellular component",
  "gene_name": "Serum amyloid A-4 protein"
}